{
  "term_label": "SCF-dependent proteasomal ubiquitin-dependent protein catabolic process",
  "gene": "UniProtKB:Q9UKA1",
  "gene_symbol": "FBXL5",
  "term_id": "GO:0031146",
  "gene_name": "F-box_LRR-repeat protein 5"
}